{
  "term_label": "extracellular space",
  "term_id": "GO:0005615",
  "gene_symbol": "A0A2R8Y747",
  "gene_name": "Uncharacterized protein",
  "gene": "UniProtKB:A0A2R8Y747"
}